formaldehyde metabolic process [GO:0046292] (biological process) Subtypes: formaldehyde assimilation [GO:0019649], formaldehyde biosynthetic process [GO:0046293], formaldehyde catabolic process [GO:0046294] Relationships: is a type of GO:0006081; is a type of GO:0044281 Sources: GOC:ai Definition: The chemical reactions and pathways involving formaldehyde (methanal, H2C=O), a colorless liquid or gas with a pungent odor, commonly used as a fixative or an antibacterial agent. Also known as: formaldehyde metabolism, methanal metabolic process, methanal metabolism